{
  "term_label": "cytoplasm",
  "gene": "UniProtKB:P13693",
  "gene_name": "Translationally-controlled tumor protein",
  "gene_symbol": "TPT1",
  "term_id": "GO:0005737"
}